{
  "gene_symbol": "DDX3X",
  "gene_name": "ATP-dependent RNA helicase DDX3X",
  "gene": "UniProtKB:O00571",
  "term_label": "mRNA binding",
  "term_id": "GO:0003729"
}